modification of postsynaptic actin cytoskeleton [GO:0098885] (biological process) Sources: GOC:dos Also known as: postsynaptic actin cytoskeleton remodelling Relationships: is a type of modification of postsynaptic structure [GO:0099010] Note: This class does not cover assembly or disassembly of synapses, only the modification/remodelling of existing ones. Definition: Any process that modifies the structure of a postsynaptic actin cytoskeleton. Regulation: regulated by GO:1905274